{
  "gene": "UniProtKB:Q05513",
  "term_id": "GO:0030010",
  "term_label": "establishment of cell polarity",
  "gene_symbol": "PRKCZ",
  "gene_name": "Protein kinase C zeta type"
}